{
  "gene": "UniProtKB:Q6XR72",
  "term_id": "GO:0005385",
  "gene_symbol": "SLC30A10",
  "term_label": "zinc ion transmembrane transporter activity",
  "gene_name": "Calcium_manganese antiporter SLC30A10"
}